{
  "gene_name": "Ras and Rab interactor 3",
  "gene_symbol": "RIN3",
  "gene": "UniProtKB:Q8TB24",
  "term_label": "guanyl-nucleotide exchange factor activity",
  "term_id": "GO:0005085"
}